allene oxide synthase activity [GO:0009978] (molecular function) References: PMID:9778849 Sources: EC:4.2.1.92 Definition: Catalysis of the reaction: 13(S)-hydroperoxylinolenate = 12,13(S)-epoxylinolenate + H2O. Also known as: (9Z,11E,14Z)-(13S)-hydroperoxyoctadeca-9,11,14-trienoate 12,13-hydro-lyase [(9Z)-(13S)-12,13-epoxyoctadeca-9,11-dienoate-forming], (9Z,11E,14Z)-(13S)-hydroperoxyoctadeca-9,11,14-trienoate 12,13-hydro-lyase activity, HPI, hydroperoxide dehydratase activity, hydroperoxide isomerase activity, linoleate hydroperoxide isomerase, linoleic acid hydroperoxide isomerase Relationships: is a type of hydro-lyase activity [GO:0016836]